{
  "term_label": "presynaptic membrane",
  "gene": "UniProtKB:Q9UJD0",
  "gene_name": "Regulating synaptic membrane exocytosis protein 3",
  "term_id": "GO:0042734",
  "gene_symbol": "RIMS3"
}